{
  "gene": "UniProtKB:P02751",
  "term_id": "GO:0005178",
  "gene_name": "Fibronectin",
  "term_label": "integrin binding",
  "gene_symbol": "FN1"
}